{
  "term_label": "Unknown cellular component",
  "gene": "UniProtKB:Q3LI73",
  "gene_name": "Keratin-associated protein 19-4",
  "term_id": "UNKNOWN:0003",
  "gene_symbol": "KRTAP19-4"
}